{
  "term_label": "glutamatergic synapse",
  "gene_name": "Leucine-rich repeat-containing protein 4C",
  "term_id": "GO:0098978",
  "gene": "UniProtKB:Q9HCJ2",
  "gene_symbol": "LRRC4C"
}